response to tumor necrosis factor [GO:0034612] (BP) Relationships: is a type of response to cytokine [GO:0034097] Subtypes: cellular response to tumor necrosis factor [GO:0071356] Also known as: response to TNF Sources: GOC:mah Definition: Any process that results in a change in state or activity of a cell or an organism (in terms of movement, secretion, enzyme production, gene expression, etc.) as a result of a tumor necrosis factor stimulus.